maintenance of left sidedness [GO:0061969] (biological process) Definition: The organization process that preserves the left sidedness in an organism's body plan or part of an organism with respect to the left and right halves. References: PMID:18629866 Sources: GOC:BHF Relationships: is a type of GO:0061968